{
  "gene_name": "Speedy protein E4",
  "term_label": "Unknown cellular component",
  "term_id": "UNKNOWN:0003",
  "gene_symbol": "SPDYE4",
  "gene": "UniProtKB:A6NLX3"
}